dehydroascorbic acid transport [GO:0070837] (biological process) Definition: The directed movement of dehydroascorbate into, out of or within a cell, or between cells, by means of some agent such as a transporter or pore. Dehydroascorbate, 5-(1,2-dihydroxyethyl)furan-2,3,4(5H)-trione, is an oxidized form of vitamin C. Sources: GOC:sl Also known as: dehydroascorbate transport Relationships: is a type of organic anion transport [GO:0015711]; is a type of vitamin transport [GO:0051180]